positive regulation of heart rate by circulating norepinephrine [GO:0003114] (biological process) Sources: GOC:mtg_cardio Definition: The process in which the secretion of norepinephrine into the bloodstream increases the rate of heart muscle contraction. Also known as: positive regulation of heart rate by circulating noradrenaline Relationships: is a type of positive regulation of heart rate by norepinephrine [GO:0003066]